{
  "term_label": "tRNA pseudouridine synthesis",
  "gene_symbol": "PUS3",
  "gene": "UniProtKB:Q9BZE2",
  "gene_name": "tRNA pseudouridine(38_39) synthase",
  "term_id": "GO:0031119"
}